versiconal hemiacetal acetate esterase activity [GO:0140397] (molecular function) Relationships: is a type of hydrolase activity, acting on ester bonds [GO:0016788] Definition: Catalyzes the reactions: versiconal hemiacetal acetate + H2O = versiconal + acetate, as well as versiconol acetate + H2O = versiconol + acetate. References: PMID:15006741, PMID:15932995, PMID:8368837 Sources: EC:3.1.1.94